{
  "gene_name": "[F-actin]-monooxygenase MICAL2",
  "gene_symbol": "MICAL2",
  "gene": "UniProtKB:O94851",
  "term_label": "oxidoreductase activity, acting on paired donors, with incorporation or reduction of molecular oxygen, NAD(P)H as one donor, and incorporation of one atom of oxygen",
  "term_id": "GO:0016709"
}